{
  "gene_symbol": "SYT12",
  "term_label": "exocytic vesicle",
  "gene": "UniProtKB:Q8IV01",
  "term_id": "GO:0070382",
  "gene_name": "Synaptotagmin-12"
}